{
  "term_id": "GO:0005730",
  "gene": "UniProtKB:Q8N567",
  "term_label": "nucleolus",
  "gene_name": "Zinc finger CCHC domain-containing protein 9",
  "gene_symbol": "ZCCHC9"
}